{
  "gene_symbol": "EEF1G",
  "gene": "UniProtKB:P26641",
  "term_id": "UNKNOWN:0001",
  "gene_name": "Elongation factor 1-gamma",
  "term_label": "Unknown molecular function"
}